extrinsic component of plastid inner membrane [GO:0035453] (cellular component) Definition: The component of a plastid inner membrane consisting of gene products and protein complexes that are loosely bound to one of its surfaces, but not integrated into the hydrophobic region. Relationships: is a type of GO:0035452; is part of GO:0009528 Sources: GOC:bf, GOC:dos Subtypes: GO:0035450 Also known as: peripheral to plastid inner membrane, extrinsic to plastid inner membrane